{
  "gene_name": "Olfactory receptor 4C46",
  "term_label": "plasma membrane",
  "gene_symbol": "OR4C46",
  "gene": "UniProtKB:A6NHA9",
  "term_id": "GO:0005886"
}